{
  "gene": "UniProtKB:Q9NQ50",
  "gene_name": "Large ribosomal subunit protein mL40",
  "term_id": "UNKNOWN:0001",
  "gene_symbol": "MRPL40",
  "term_label": "Unknown molecular function"
}